{
  "gene_name": "Mothers against decapentaplegic homolog 6",
  "gene_symbol": "SMAD6",
  "term_label": "SMAD protein signal transduction",
  "term_id": "GO:0060395",
  "gene": "UniProtKB:O43541"
}